signal transduction involved in regulation of gene expression [GO:0023019] (biological process) Relationships: is a type of signal transduction [GO:0007165]; is part of GO:0010468 Also known as: regulation of gene expression as a consequence of signal transmission Sources: GOC:mtg_signal Definition: Any process that modulates the frequency, rate or extent of gene expression as a consequence of a process in which a signal is released and/or conveyed from one location to another.